{
  "gene": "UniProtKB:Q96IR2",
  "term_label": "transcription cis-regulatory region binding",
  "gene_symbol": "ZNF845",
  "gene_name": "Zinc finger protein 845",
  "term_id": "GO:0000976"
}